{
  "term_id": "GO:0005615",
  "term_label": "extracellular space",
  "gene": "UniProtKB:O76093",
  "gene_name": "Fibroblast growth factor 18",
  "gene_symbol": "FGF18"
}